{
  "gene_name": "Dystroglycan 1",
  "term_id": "GO:0007411",
  "term_label": "axon guidance",
  "gene": "UniProtKB:Q14118",
  "gene_symbol": "DAG1"
}